{
  "gene_symbol": "DONSON",
  "gene": "UniProtKB:Q9NYP3",
  "term_id": "GO:0005634",
  "term_label": "nucleus",
  "gene_name": "Protein downstream neighbor of Son"
}